{
  "gene_name": "DNA-binding protein RFX6",
  "term_id": "GO:0006357",
  "gene": "UniProtKB:Q8HWS3",
  "gene_symbol": "RFX6",
  "term_label": "regulation of transcription by RNA polymerase II"
}